{
  "gene_name": "Ras-related protein Ral-A",
  "term_id": "GO:0003924",
  "gene_symbol": "RALA",
  "term_label": "GTPase activity",
  "gene": "UniProtKB:P11233"
}